actin cytoskeleton organization [GO:0030036] (BP) Regulation: regulated by GO:0032956 Relationships: is a type of cytoskeleton organization [GO:0007010]; is a type of actin filament-based process [GO:0030029] Sources: GOC:dph, GOC:jl, GOC:mah Subtypes: GO:0030047, cortical actin cytoskeleton organization [GO:0030866], establishment or maintenance of actin cytoskeleton polarity [GO:0030950], actomyosin structure organization [GO:0031032], myosin filament organization [GO:0031033], paramyosin filament assembly or disassembly [GO:0061204], postsynaptic actin cytoskeleton organization [GO:0098974], presynaptic actin cytoskeleton organization [GO:0099140], GO:1904600 Definition: A process that is carried out at the cellular level which results in the assembly, arrangement of constituent parts, or disassembly of cytoskeletal structures comprising actin filaments and their associated proteins. Also known as: actin cytoskeleton organisation, actin cytoskeleton organization and biogenesis, actin modulating activity